{
  "term_label": "thiamine transmembrane transporter activity",
  "term_id": "GO:0015234",
  "gene": "UniProtKB:Q9HC21",
  "gene_name": "Mitochondrial thiamine pyrophosphate carrier",
  "gene_symbol": "SLC25A19"
}